{
  "term_id": "UNKNOWN:0001",
  "term_label": "Unknown molecular function",
  "gene": "UniProtKB:Q3LI68",
  "gene_symbol": "KRTAP22-2",
  "gene_name": "Keratin-associated protein 22-2"
}